{
  "term_label": "Unknown molecular function",
  "gene_name": "Integrator complex subunit 7",
  "gene_symbol": "INTS7",
  "gene": "UniProtKB:Q9NVH2",
  "term_id": "UNKNOWN:0001"
}